{
  "gene_symbol": "CPEB3",
  "term_label": "cytoplasm",
  "gene_name": "Cytoplasmic polyadenylation element-binding protein 3",
  "gene": "UniProtKB:Q8NE35",
  "term_id": "GO:0005737"
}